{
  "term_label": "Unknown biological process",
  "gene_symbol": "MCOLN3",
  "gene_name": "Mucolipin-3",
  "term_id": "UNKNOWN:0002",
  "gene": "UniProtKB:Q8TDD5"
}